{
  "gene_symbol": "TSHZ1",
  "gene_name": "Teashirt homolog 1",
  "term_id": "GO:0000981",
  "gene": "UniProtKB:Q6ZSZ6",
  "term_label": "DNA-binding transcription factor activity, RNA polymerase II-specific"
}